{
  "term_label": "Unknown cellular component",
  "gene": "UniProtKB:Q9H6N6",
  "gene_name": "Putative uncharacterized protein MYH16",
  "term_id": "UNKNOWN:0003",
  "gene_symbol": "MYH16"
}